{
  "term_id": "UNKNOWN:0002",
  "gene_name": "N6-adenosine-methyltransferase TMT1A",
  "gene": "UniProtKB:Q9H8H3",
  "gene_symbol": "TMT1A",
  "term_label": "Unknown biological process"
}